{
  "term_id": "GO:0031410",
  "gene": "UniProtKB:Q92738",
  "gene_symbol": "USP6NL",
  "term_label": "cytoplasmic vesicle",
  "gene_name": "USP6 N-terminal-like protein"
}